{
  "gene_name": "Ephrin type-A receptor 7",
  "term_id": "GO:0007411",
  "gene_symbol": "EPHA7",
  "gene": "UniProtKB:Q15375",
  "term_label": "axon guidance"
}